{
  "term_id": "UNKNOWN:0003",
  "gene": "UniProtKB:Q13761",
  "term_label": "Unknown cellular component",
  "gene_name": "Runt-related transcription factor 3",
  "gene_symbol": "RUNX3"
}